{
  "gene_name": "Serine-rich coiled-coil domain-containing protein 2",
  "gene": "UniProtKB:Q9H7U1",
  "gene_symbol": "CCSER2",
  "term_id": "GO:0008017",
  "term_label": "microtubule binding"
}